{
  "gene_name": "Ras-related protein M-Ras",
  "term_label": "plasma membrane",
  "gene": "UniProtKB:O14807",
  "gene_symbol": "MRAS",
  "term_id": "GO:0005886"
}